epithelial cell migration involved in mesonephric nephron tubule morphogenesis [GO:0061278] (biological process) Sources: GOC:mtg_kidney_jan10 Subtypes: epithelial cell migration involved in mesonephric distal tubule morphogenesis [GO:0061279], epithelial cell migration involved in mesonephric proximal tubule morphogenesis [GO:0061280] Definition: The orderly movement of epithelial cells within a renal tubule that contributes to mesonephric nephron tubule morphogenesis. Relationships: is a type of epithelial cell migration involved in nephron tubule morphogenesis [GO:0072155]; BFO_0000050 mesonephric nephron tubule morphogenesis [GO:0061240]